{
  "gene": "UniProtKB:O00625",
  "gene_symbol": "PIR",
  "term_label": "quercetin 2,3-dioxygenase activity",
  "gene_name": "Pirin",
  "term_id": "GO:0008127"
}